{
  "term_id": "GO:0009897",
  "gene_symbol": "CD24",
  "gene": "UniProtKB:P25063",
  "gene_name": "Signal transducer CD24",
  "term_label": "external side of plasma membrane"
}